{
  "gene": "UniProtKB:O75525",
  "term_label": "nucleus",
  "gene_symbol": "KHDRBS3",
  "term_id": "GO:0005634",
  "gene_name": "KH domain-containing, RNA-binding, signal transduction-associated protein 3"
}